xanthophore [GO:0031633] (cellular component) Definition: A chromatophore containing yellow pigment. Sources: ISBN:0395825172 Relationships: is a type of plasma membrane-derived chromatophore [GO:0042716] Note: Note that this term refers to a subcellular structure, and should not be confused with the specialized cells known as xanthophores, which produce yellow pigment and are found in fish and amphibian skin. Note that several terms in the biological process ontology ('xanthophore differentiation ; GO:0050936' and its children) refer to xanthophores in the sense of pigment-producing cells.